{
  "term_id": "GO:0001181",
  "gene_name": "RNA polymerase I-specific transcription initiation factor RRN3",
  "gene_symbol": "RRN3",
  "gene": "UniProtKB:Q9NYV6",
  "term_label": "RNA polymerase I general transcription initiation factor activity"
}